{
  "gene_symbol": "RERG",
  "gene": "UniProtKB:Q96A58",
  "term_label": "plasma membrane",
  "gene_name": "Ras-related and estrogen-regulated growth inhibitor",
  "term_id": "GO:0005886"
}